mRNA 3'-end processing [GO:0031124] (biological process) Regulation: regulated by regulation of mRNA 3'-end processing [GO:0031440]; negatively regulated by GO:0031441; positively regulated by positive regulation of mRNA 3'-end processing [GO:0031442] Relationships: is a type of mRNA processing [GO:0006397]; is_a RNA 3'-end processing [GO:0031123] Definition: Any process involved in forming the mature 3' end of an mRNA molecule. Also known as: mRNA 3' end processing Subtypes: mRNA 3'-end processing by stem-loop binding and cleavage [GO:0006398], mitochondrial mRNA 3'-end processing [GO:0090616], GO:0110104, co-transcriptional mRNA 3'-end processing, cleavage and polyadenylation pathway [GO:0180010] Sources: GOC:mah